aldehyde oxygenase (deformylating) activity [GO:0071771] (MF) Also known as: aldehyde decarbonylase activity, decarbonylase activity Definition: Catalysis of the reaction: a long-chain fatty aldehyde + H+ + 2 NADPH + O2 = a long-chain alkane + formate + H2O + 2 NADP+. References: PMID:6593720, PMID:8718622 Sources: RHEA:21440 Relationships: is a type of carbon-carbon lyase activity [GO:0016830]